{
  "term_id": "UNKNOWN:0001",
  "gene_symbol": "TNFRSF10D",
  "gene_name": "Tumor necrosis factor receptor superfamily member 10D",
  "gene": "UniProtKB:Q9UBN6",
  "term_label": "Unknown molecular function"
}